axon hillock [GO:0043203] (cellular component) Definition: Portion of the neuronal cell soma from which the axon originates. Relationships: is a type of cellular anatomical structure [GO:0110165]; is part of axon [GO:0030424]; is part of neuronal cell body [GO:0043025] Sources: GOC:nln